{
  "gene_name": "Spindle and kinetochore-associated protein 3",
  "gene_symbol": "SKA3",
  "term_label": "Unknown molecular function",
  "term_id": "UNKNOWN:0001",
  "gene": "UniProtKB:Q8IX90"
}